{
  "term_id": "UNKNOWN:0001",
  "gene_name": "P-selectin glycoprotein ligand 1",
  "gene_symbol": "SELPLG",
  "gene": "UniProtKB:Q14242",
  "term_label": "Unknown molecular function"
}